{
  "term_label": "Unknown molecular function",
  "term_id": "UNKNOWN:0001",
  "gene_name": "Putative uncharacterized protein LOC400499",
  "gene_symbol": "Q6ZTK2",
  "gene": "UniProtKB:Q6ZTK2"
}